arabinoxylan-containing compound catabolic process [GO:2000888] (biological process) Relationships: is a type of xylan catabolic process [GO:0045493] Definition: The chemical reactions and pathways resulting in the breakdown of an arabinoxylan. Sources: GOC:mengo_curators Subtypes: GO:2000887 Also known as: arabinoxylan catabolic process, arabinoxylan catabolism Regulation: regulated by GO:2000921; negatively regulated by negative regulation of arabinoxylan-containing compound catabolic process [GO:2000922]; positively regulated by positive regulation of arabinoxylan-containing compound catabolic process [GO:2000923]